{
  "term_id": "GO:0000977",
  "term_label": "RNA polymerase II transcription regulatory region sequence-specific DNA binding",
  "gene": "UniProtKB:Q9NU63",
  "gene_symbol": "ZFP57",
  "gene_name": "Zinc finger protein 57 homolog"
}